regulation of anti-Mullerian hormone signaling pathway [GO:1902612] (biological process) Definition: Any process that modulates the frequency, rate or extent of anti-Mullerian hormone signaling pathway. Subtypes: negative regulation of anti-Mullerian hormone signaling pathway [GO:1902613], positive regulation of anti-Mullerian hormone signaling pathway [GO:1902614] References: PMID:23624077 Sources: GOC:TermGenie, GOC:hjd, GO_REF:0000058 Relationships: is a type of regulation of transmembrane receptor protein serine/threonine kinase signaling pathway [GO:0090092]; regulates anti-Mullerian hormone receptor signaling pathway [GO:1990262]